{
  "term_id": "GO:0001609",
  "gene_name": "Adenosine receptor A1",
  "term_label": "G protein-coupled adenosine receptor activity",
  "gene_symbol": "ADORA1",
  "gene": "UniProtKB:P30542"
}